pituitary gland development [GO:0021983] (biological process) Relationships: is a type of GO:0048732; is part of diencephalon development [GO:0021536]; is part of endocrine system development [GO:0035270] Also known as: hypophysis development Definition: The progression of the pituitary gland over time from its initial formation until its mature state. The pituitary gland is an endocrine gland that secretes hormones that regulate many other glands. Sources: GOC:cls, GOC:dgh, GOC:dph, GOC:jid, GO_REF:0000021